{
  "term_id": "GO:0015020",
  "gene_name": "UDP-glucuronosyltransferase 2B11",
  "gene": "UniProtKB:O75310",
  "term_label": "glucuronosyltransferase activity",
  "gene_symbol": "UGT2B11"
}